{
  "gene_name": "UPF0669 protein C6orf120",
  "term_label": "Unknown molecular function",
  "gene_symbol": "C6orf120",
  "term_id": "UNKNOWN:0001",
  "gene": "UniProtKB:Q7Z4R8"
}